forebrain neuron development [GO:0021884] (biological process) Definition: The process whose specific outcome is the progression of a neuron that resides in the forebrain, from its initial commitment to its fate, to the fully functional differentiated cell. Sources: GOC:cls, GOC:dgh, GOC:dph, GOC:jid, GO_REF:0000021 Relationships: is_a GO:0021954; is part of forebrain neuron differentiation [GO:0021879] Subtypes: GO:0021860, hypothalamus gonadotrophin-releasing hormone neuron development [GO:0021888], olfactory bulb interneuron development [GO:0021891], cerebral cortex GABAergic interneuron development [GO:0021894], thyroid-stimulating hormone-secreting cell development [GO:0060130], olfactory bulb tufted cell development [GO:0061449]